{
  "gene_name": "Neuronal acetylcholine receptor subunit beta-3",
  "term_label": "membrane depolarization",
  "term_id": "GO:0051899",
  "gene_symbol": "CHRNB3",
  "gene": "UniProtKB:Q05901"
}